malic acid secretion [GO:0046723] (BP) Sources: GOC:ai Definition: The controlled release of malic acid, hydroxybutanedioic (hydroxysuccinic) acid, by a cell or a tissue. Also known as: hydroxysuccinic acid secretion, malate secretion Relationships: is a type of malate transport [GO:0015743]; is a type of acid secretion [GO:0046717]